negative regulation of execution phase of apoptosis [GO:1900118] (biological process) Subtypes: GO:1905781 Relationships: is a type of GO:0043066; is a type of GO:1900117; negatively regulates execution phase of apoptosis [GO:0097194] Also known as: down regulation of execution phase of apoptosis, down-regulation of execution phase of apoptosis, downregulation of execution phase of apoptosis, inhibition of execution phase of apoptosis Sources: GOC:TermGenie, GOC:mtg_apoptosis Definition: Any process that stops, prevents or reduces the frequency, rate or extent of execution phase of apoptosis.